regulation of sulfur utilization [GO:0006792] (BP) Relationships: is a type of GO:0032107; RO_0002211 sulfur utilization [GO:0006791] Sources: GOC:go_curators Subtypes: negative regulation of sulfur utilization [GO:0045882], GO:0045883 Also known as: regulation of sulphur utilization Definition: Any process that modulates the frequency, rate or extent of sulfur utilization.